{
  "term_id": "GO:0098609",
  "term_label": "cell-cell adhesion",
  "gene_symbol": "ITGA8",
  "gene_name": "Integrin alpha-8",
  "gene": "UniProtKB:P53708"
}